endoplasmic reticulum-derived vesicle fusion with endoplasmic reticulum-Golgi intermediate compartment (ERGIC) membrane [GO:1990687] (BP) Relationships: is a type of vesicle fusion with endoplasmic reticulum-Golgi intermediate compartment (ERGIC) membrane [GO:1990668]; is part of endoplasmic reticulum to Golgi vesicle-mediated transport [GO:0006888] References: PMID:16038056, PMID:24119662 Sources: GOC:bhm Also known as: ER-derived vesicle fusion with ER-Golgi intermediate compartment membrane, ER-derived vesicle fusion with ERGIC membrane Definition: The joining of the lipid bilayer membrane around an endoplasmic reticulum-derived vesicle to the lipid bilayer membrane of the ERGIC. Such vesicles include COPII-coated transport vesicles involved in anterograde transport.